{
  "term_id": "UNKNOWN:0003",
  "gene": "UniProtKB:Q8N5V2",
  "gene_symbol": "NGEF",
  "term_label": "Unknown cellular component",
  "gene_name": "Ephexin-1"
}